{
  "term_id": "GO:0002020",
  "gene": "UniProtKB:P78560",
  "gene_name": "Death domain-containing protein CRADD",
  "gene_symbol": "CRADD",
  "term_label": "protease binding"
}